ventral midline development [GO:0007418] (biological process) Definition: The process whose specific outcome is the progression of the ventral midline over time, from its formation to the mature structure. In protostomes (such as insects, snails and worms) as well as deuterostomes (vertebrates), the midline is an embryonic region that functions in patterning of the adjacent nervous tissue. The ventral midline in insects is a cell population extending along the ventral surface of the embryo and is the region from which cells detach to form the ventrally located nerve cords. In vertebrates, the midline is originally located dorsally. During development, it folds inwards and becomes the ventral part of the dorsally located neural tube and is then called the ventral midline, or floor plate. References: PMID:12075342 Sources: GOC:bf, GOC:go_curators Relationships: is a type of GO:0048856; is part of GO:0007417